host cell endosome [GO:0044174] (cellular component) Definition: A membrane-bounded organelle that carries materials newly ingested by endocytosis. It passes many of the materials to host cell lysosomes for degradation. Sources: GOC:jl Relationships: is a type of host intracellular membrane-bounded organelle [GO:0033648]; is a type of host cell cytoplasm part [GO:0033655] Also known as: host endosome Subtypes: host cell late endosome [GO:0044184]